meiotic DNA integrity checkpoint signaling [GO:0044778] (biological process) Subtypes: GO:0033315 Definition: A signal transduction process that controls cell cycle progression in response to changes in DNA structure by monitoring the integrity of the DNA during meiosis. The DNA integrity checkpoint begins with detection of DNA damage, defects in DNA structure or DNA replication, and ends with signal transduction. Also known as: meiotic DNA integrity checkpoint Relationships: is a type of DNA integrity checkpoint signaling [GO:0031570]; is a type of meiotic cell cycle checkpoint signaling [GO:0033313] Sources: GOC:mtg_cell_cycle